{
  "gene_name": "ATP-dependent zinc metalloprotease YME1L1",
  "gene_symbol": "YME1L1",
  "term_label": "mitochondrial inner membrane",
  "term_id": "GO:0005743",
  "gene": "UniProtKB:Q96TA2"
}